{
  "term_label": "nucleus",
  "gene_name": "Structural maintenance of chromosomes protein 6",
  "gene_symbol": "SMC6",
  "term_id": "GO:0005634",
  "gene": "UniProtKB:Q96SB8"
}